{
  "term_id": "GO:0070301",
  "gene_name": "Peptidyl-prolyl cis-trans isomerase F, mitochondrial",
  "gene": "UniProtKB:P30405",
  "term_label": "cellular response to hydrogen peroxide",
  "gene_symbol": "PPIF"
}